{
  "gene_name": "Protein arginine N-methyltransferase 1",
  "term_id": "GO:0005634",
  "term_label": "nucleus",
  "gene": "UniProtKB:Q99873",
  "gene_symbol": "PRMT1"
}